{
  "gene": "UniProtKB:Q8WWG9",
  "term_id": "GO:0005251",
  "gene_name": "Potassium voltage-gated channel subfamily E member 4",
  "gene_symbol": "KCNE4",
  "term_label": "delayed rectifier potassium channel activity"
}